{
  "gene_symbol": "TNRC18",
  "term_id": "UNKNOWN:0003",
  "gene_name": "Trinucleotide repeat-containing gene 18 protein",
  "term_label": "Unknown cellular component",
  "gene": "UniProtKB:O15417"
}